{
  "gene_name": "Putative protein LRRC37A5P",
  "term_label": "Unknown biological process",
  "term_id": "UNKNOWN:0002",
  "gene": "UniProtKB:Q49AS3",
  "gene_symbol": "LRRC37A5P"
}